{
  "term_label": "indoleamine 2,3-dioxygenase activity",
  "gene_name": "Indoleamine 2,3-dioxygenase 2",
  "term_id": "GO:0033754",
  "gene": "UniProtKB:Q6ZQW0",
  "gene_symbol": "IDO2"
}